{
  "gene_symbol": "EEPD1",
  "term_label": "plasma membrane",
  "gene_name": "Endonuclease_exonuclease_phosphatase family domain-containing protein 1",
  "term_id": "GO:0005886",
  "gene": "UniProtKB:Q7L9B9"
}